{
  "gene": "UniProtKB:P51801",
  "term_label": "chloride transport",
  "term_id": "GO:0006821",
  "gene_symbol": "CLCNKB",
  "gene_name": "Chloride channel protein ClC-Kb"
}